{
  "term_label": "UDP-glycosyltransferase activity",
  "gene_name": "UDP-glucuronosyltransferase 1A3",
  "term_id": "GO:0008194",
  "gene": "UniProtKB:P35503",
  "gene_symbol": "UGT1A3"
}